{
  "gene_symbol": "HPDL",
  "gene_name": "4-hydroxyphenylpyruvate dioxygenase-like protein",
  "gene": "UniProtKB:Q96IR7",
  "term_label": "Unknown biological process",
  "term_id": "UNKNOWN:0002"
}